response to ionomycin [GO:1904636] (biological process) Definition: Any process that results in a change in state or activity of a cell or an organism (in terms of movement, secretion, enzyme production, gene expression, etc.) as a result of an ionomycin stimulus. References: PMID:17516843 Sources: GOC:TermGenie, GO_REF:0000071 Relationships: is a type of response to ether [GO:0045472]; is a type of response to fatty acid [GO:0070542] Subtypes: cellular response to ionomycin [GO:1904637]